{
  "term_id": "GO:0005759",
  "gene": "UniProtKB:A0A8I5KW96",
  "gene_name": "Adenylate kinase 4, mitochondrial",
  "gene_symbol": "AK4P3",
  "term_label": "mitochondrial matrix"
}